{
  "term_id": "GO:0050772",
  "gene": "UniProtKB:Q9ULL4",
  "gene_symbol": "PLXNB3",
  "gene_name": "Plexin-B3",
  "term_label": "positive regulation of axonogenesis"
}